androgen biosynthetic process [GO:0006702] (biological process) Regulation: negatively regulated by negative regulation of androgen biosynthetic process [GO:2000180] Also known as: androgen anabolism, androgen biosynthesis, androgen formation, androgen synthesis Sources: ISBN:0198506732 Definition: The chemical reactions and pathways resulting in the formation of androgens, C19 steroid hormones that can stimulate the development of male sexual characteristics. Relationships: is a type of androgen metabolic process [GO:0008209]; is a type of GO:0042446; is a type of steroid hormone biosynthetic process [GO:0120178]